{
  "term_id": "GO:0005634",
  "term_label": "nucleus",
  "gene_symbol": "NR4A3",
  "gene": "UniProtKB:Q92570",
  "gene_name": "Nuclear receptor subfamily 4 group A member 3"
}